{
  "gene": "UniProtKB:A4D1E1",
  "term_label": "Unknown biological process",
  "term_id": "UNKNOWN:0002",
  "gene_name": "Zinc finger protein 804B",
  "gene_symbol": "ZNF804B"
}